{
  "term_id": "UNKNOWN:0001",
  "gene_name": "Mucin-like protein 1",
  "term_label": "Unknown molecular function",
  "gene": "UniProtKB:Q96DR8",
  "gene_symbol": "MUCL1"
}